{
  "term_id": "GO:0031647",
  "gene_name": "Ubiquitin carboxyl-terminal hydrolase 17-like protein 1",
  "term_label": "regulation of protein stability",
  "gene": "UniProtKB:Q7RTZ2",
  "gene_symbol": "USP17L1"
}